{
  "gene_name": "RING finger protein 212B",
  "gene_symbol": "RNF212B",
  "term_id": "GO:0007129",
  "term_label": "homologous chromosome pairing at meiosis",
  "gene": "UniProtKB:A8MTL3"
}